{
  "gene_name": "Signal transducer and activator of transcription 1-alpha_beta",
  "gene_symbol": "STAT1",
  "term_label": "ISGF3 complex",
  "term_id": "GO:0070721",
  "gene": "UniProtKB:P42224"
}